{
  "gene": "UniProtKB:O75820",
  "gene_symbol": "ZNF189",
  "term_id": "GO:0000978",
  "term_label": "RNA polymerase II cis-regulatory region sequence-specific DNA binding",
  "gene_name": "Zinc finger protein 189"
}